{
  "gene_symbol": "MALSU1",
  "gene": "UniProtKB:Q96EH3",
  "gene_name": "Mitochondrial assembly of ribosomal large subunit protein 1",
  "term_label": "ribosomal large subunit binding",
  "term_id": "GO:0043023"
}